{
  "gene_name": "Uridine phosphorylase 1",
  "term_id": "GO:0005829",
  "term_label": "cytosol",
  "gene_symbol": "UPP1",
  "gene": "UniProtKB:Q16831"
}